brush border assembly [GO:1904970] (biological process) References: PMID:24725409 Sources: GOC:TermGenie, GOC:lb, GO_REF:0000079 Relationships: is a type of cellular component assembly [GO:0022607] Definition: The aggregation, arrangement and bonding together of adjacent microvilli through the formation of Ca(2+)-dependent adhesion links between them, forming a brush border. Also known as: brush border formation